{
  "term_id": "GO:0005634",
  "gene": "UniProtKB:Q00535",
  "term_label": "nucleus",
  "gene_symbol": "CDK5",
  "gene_name": "Cyclin-dependent kinase 5"
}